{
  "gene": "UniProtKB:Q9P2G9",
  "gene_symbol": "KLHL8",
  "term_label": "proteasome-mediated ubiquitin-dependent protein catabolic process",
  "term_id": "GO:0043161",
  "gene_name": "Kelch-like protein 8"
}